{
  "term_id": "GO:0005009",
  "gene_name": "Insulin receptor",
  "gene_symbol": "INSR",
  "term_label": "insulin receptor activity",
  "gene": "UniProtKB:P06213"
}